{
  "gene_name": "Lipocalin_cytosolic fatty-acid binding domain-containing protein",
  "gene_symbol": "LOC102723971",
  "term_id": "GO:0005615",
  "term_label": "extracellular space",
  "gene": "UniProtKB:A0A1B0GUV8"
}